{
  "gene_name": "Erlin-1",
  "gene_symbol": "ERLIN1",
  "term_id": "GO:0015485",
  "term_label": "cholesterol binding",
  "gene": "UniProtKB:O75477"
}